transferase activity, transferring sulphur-containing groups [GO:0016782] (molecular function) Definition: Catalysis of the transfer of a sulfur-containing group from one compound (donor) to another (acceptor). Sources: EC:2.8.-.- Relationships: is a type of transferase activity [GO:0016740] Subtypes: sulfotransferase activity [GO:0008146], GO:0008410, sulfurtransferase activity [GO:0016783], iron-sulfur transferase activity [GO:0036455], alkylthioltransferase activity [GO:0050497]